{
  "term_id": "GO:0005886",
  "term_label": "plasma membrane",
  "gene_symbol": "EMB",
  "gene_name": "Embigin",
  "gene": "UniProtKB:Q6PCB8"
}